{
  "gene_symbol": "ADM",
  "term_id": "GO:0031700",
  "gene_name": "Pro-adrenomedullin",
  "term_label": "adrenomedullin receptor binding",
  "gene": "UniProtKB:P35318"
}